negative regulation of muscle atrophy [GO:0014736] (BP) Definition: Any process that stops, prevents, or reduces the frequency, rate, or extent of muscle atrophy. Relationships: is a type of regulation of muscle atrophy [GO:0014735]; is a type of negative regulation of muscle adaptation [GO:0014745]; negatively regulates muscle atrophy [GO:0014889] Sources: GOC:mtg_muscle